renal sodium ion absorption involved in negative regulation of renal sodium excretion [GO:0035817] (biological process) Definition: Any process where sodium ions are taken up from the collecting ducts and proximal and distal loops of the nephron, which contributes to decreasing the amount of sodium that is excreted in urine per unit time. Relationships: is a type of renal sodium ion absorption [GO:0070294]; is part of negative regulation of renal sodium excretion [GO:0035814] Sources: GOC:mtg_25march11, GOC:yaf